{
  "gene_name": "Unconventional myosin-Vc",
  "term_label": "actin cytoskeleton",
  "gene_symbol": "MYO5C",
  "gene": "UniProtKB:Q9NQX4",
  "term_id": "GO:0015629"
}